regulation of mitotic recombination-dependent replication fork processing [GO:1903221] (biological process) References: PMID:23093942 Sources: GOC:TermGenie, GO_REF:0000058 Subtypes: negative regulation of mitotic recombination-dependent replication fork processing [GO:0120291], GO:0120292 Also known as: regulation of mitotic recombination involved in collapsed replication fork processing, regulation of mitotic recombination involved in recovery from replication fork arrest, regulation of mitotic recombination involved in recovery from replication fork stalling, regulation of mitotic recombination involved in replication fork processing, prevention of genomic instability induced by DNA replication fork arrest, regulation of mitotic recombination involved in replication fork restart, regulation of mitotic recombination involved in replication restart Relationships: is a type of regulation of cell cycle process [GO:0010564]; is a type of GO:0051052; regulates mitotic recombination-dependent replication fork processing [GO:1990426] Definition: Any process that modulates the frequency, rate or extent of mitotic recombination-dependent replication fork processing. Regulation of mitotic recombination prevents recombination between inappropriate homologous sequences.